{
  "gene_symbol": "CD28",
  "gene": "UniProtKB:P10747",
  "term_id": "GO:0042110",
  "term_label": "T cell activation",
  "gene_name": "T-cell-specific surface glycoprotein CD28"
}